glycerol-3-phosphate catabolic process [GO:0046168] (biological process) Also known as: glycerol-3-phosphate breakdown, glycerol-3-phosphate catabolism, glycerol-3-phosphate degradation Definition: The chemical reactions and pathways resulting in the breakdown of glycerol-3-phosphate, a phosphoric monoester of glycerol. Sources: GOC:ai Relationships: is a type of glycerol-3-phosphate metabolic process [GO:0006072]; is a type of organophosphate catabolic process [GO:0046434]; is a type of GO:1901136